{
  "gene_symbol": "A8MUI8",
  "gene_name": "Putative UPF0607 protein ENSP00000383783",
  "term_label": "Unknown cellular component",
  "term_id": "UNKNOWN:0003",
  "gene": "UniProtKB:A8MUI8"
}